single-stranded RNA binding [GO:0003727] (MF) Sources: GOC:jl Relationships: is a type of RNA binding [GO:0003723] Subtypes: steroid receptor RNA activator RNA binding [GO:0002153], poly-pyrimidine tract binding [GO:0008187], GO:0033592, RNA strand-exchange activity [GO:0034057], poly-purine tract binding [GO:0070717] Also known as: ssRNA binding Definition: Binding to single-stranded RNA.